{
  "gene": "UniProtKB:Q9Y6I9",
  "gene_symbol": "TEX264",
  "term_label": "reticulophagy",
  "term_id": "GO:0061709",
  "gene_name": "Testis-expressed protein 264"
}